{
  "gene": "UniProtKB:Q9UHB6",
  "term_label": "actin filament bundle assembly",
  "gene_symbol": "LIMA1",
  "gene_name": "LIM domain and actin-binding protein 1",
  "term_id": "GO:0051017"
}